{
  "gene_name": "Ras-related protein Rab-9A",
  "gene": "UniProtKB:P51151",
  "gene_symbol": "RAB9A",
  "term_label": "phagocytic vesicle",
  "term_id": "GO:0045335"
}